{
  "gene": "UniProtKB:O95522",
  "gene_symbol": "PRAMEF12",
  "term_label": "ubiquitin-like ligase-substrate adaptor activity",
  "gene_name": "PRAME family member 12",
  "term_id": "GO:1990756"
}